negative regulation of gastric acid secretion [GO:0060455] (biological process) Definition: Any process that decreases the rate frequency or extent of gastric secretion. Gastric secretion is the regulated release of gastric acid (hydrochloric acid) by parietal or oxyntic cells during digestion. Sources: GOC:dph, GOC:tb Subtypes: negative regulation of gastrin-induced gastric acid secretion [GO:1903640] Relationships: is a type of negative regulation of secretion [GO:0051048]; is a type of regulation of gastric acid secretion [GO:0060453]; is a type of negative regulation of digestive system process [GO:0060457]; RO_0002212 gastric acid secretion [GO:0001696]